{
  "gene_symbol": "EGR2",
  "gene_name": "E3 SUMO-protein ligase EGR2",
  "term_id": "GO:0000978",
  "gene": "UniProtKB:P11161",
  "term_label": "RNA polymerase II cis-regulatory region sequence-specific DNA binding"
}